{
  "term_id": "GO:0005085",
  "gene_name": "Dedicator of cytokinesis protein 8",
  "term_label": "guanyl-nucleotide exchange factor activity",
  "gene": "UniProtKB:Q8NF50",
  "gene_symbol": "DOCK8"
}